{
  "term_id": "GO:0005850",
  "gene_name": "Eukaryotic translation initiation factor 2 subunit 3",
  "gene_symbol": "EIF2S3",
  "gene": "UniProtKB:P41091",
  "term_label": "eukaryotic translation initiation factor 2 complex"
}